{
  "term_label": "Unknown molecular function",
  "gene_symbol": "MEGF8",
  "gene": "UniProtKB:Q7Z7M0",
  "term_id": "UNKNOWN:0001",
  "gene_name": "Multiple epidermal growth factor-like domains protein 8"
}